{
  "gene": "UniProtKB:O43933",
  "term_label": "protein unfolding",
  "gene_symbol": "PEX1",
  "term_id": "GO:0043335",
  "gene_name": "Peroxisomal ATPase PEX1"
}